{
  "gene_symbol": "CDIPT",
  "gene": "UniProtKB:O14735",
  "term_id": "GO:0003881",
  "gene_name": "CDP-diacylglycerol--inositol 3-phosphatidyltransferase",
  "term_label": "CDP-diacylglycerol-inositol 3-phosphatidyltransferase activity"
}